hypoxanthine phosphoribosyltransferase activity [GO:0004422] (molecular function) Also known as: Transphosphoribosidase activity, guanine-hypoxanthine phosphoribosyltransferase activity, hypoxanthine-guanine phosphoribosyltransferase activity, 6-hydroxypurine phosphoribosyltransferase activity, 6-mercaptopurine phosphoribosyltransferase activity, HGPRTase activity, HPRT, IMP diphosphorylase activity, IMP pyrophosphorylase activity, IMP-GMP pyrophosphorylase activity, IMP:diphosphate phospho-D-ribosyltransferase activity, inosinate pyrophosphorylase activity, inosine 5'-phosphate pyrophosphorylase activity, inosinic acid pyrophosphorylase activity, inosinic pyrophosphorylase activity, purine-6-thiol phosphoribosyltransferase activity Sources: RHEA:17973 Relationships: is a type of GO:0106130 Definition: Catalysis of the reaction: IMP + diphosphate = hypoxanthine + 5-phospho-alpha-D-ribose 1-diphosphate.